allantoinase activity [GO:0004038] (molecular function) Definition: Catalysis of the reaction: allantoin + H2O = allantoate. Also known as: (S)-allantoin amidohydrolase activity Relationships: is a type of hydrolase activity, acting on carbon-nitrogen (but not peptide) bonds, in cyclic amides [GO:0016812] Sources: EC:3.5.2.5